{
  "term_id": "GO:0008081",
  "gene": "UniProtKB:Q6UWV6",
  "gene_name": "Ectonucleotide pyrophosphatase_phosphodiesterase family member 7",
  "gene_symbol": "ENPP7",
  "term_label": "phosphoric diester hydrolase activity"
}